{
  "term_label": "potassium ion import across plasma membrane",
  "gene_name": "Potassium channel subfamily K member 9",
  "gene_symbol": "KCNK9",
  "term_id": "GO:1990573",
  "gene": "UniProtKB:Q9NPC2"
}